keratan sulfate-II proteoglycan biosynthetic process [GO:0140264] (BP) Definition: The chemical reactions and pathways resulting in the formation of keratan sulfate II (KS-II), O-linked via a GalNAc attached to a serine or a threonine residue in the target protein. Relationships: is a type of GO:0016266; is a type of GO:0018146 Also known as: O-linked GalNAc-keratan sulfate-II proteoglycan biosynthetic process References: PMID:29340594